ecdysone-mediated polytene chromosome puffing [GO:0035077] (biological process) Definition: The decondensing (loosening) and swelling of the chromosomal sites of hormone-responsive genes on polytene chromosomes in response to increased production of the steroid hormone 20-hydroxyecdysone (ecdysone) in Drosophila larvae approaching pupation. Relationships: is a type of polytene chromosome puffing [GO:0035079]; is part of cellular response to ecdysone [GO:0071390] References: PMID:12543962 Sources: GOC:bf